response to alcohol [GO:0097305] (biological process) References: PMID:24014527 Sources: GOC:pr Subtypes: response to abscisic acid [GO:0009737], response to vitamin B1 [GO:0010266], response to methanol [GO:0033986], response to prostaglandin E [GO:0034695], response to ecdysone [GO:0035075], response to ethanol [GO:0045471], response to cycloheximide [GO:0046898], response to corticosterone [GO:0051412], response to cortisone [GO:0051413], GO:0051414, GO:0070723, response to indole-3-methanol [GO:0071680], response to prostaglandin D [GO:0071798], response to mercaptoethanol [GO:0072704], cellular response to alcohol [GO:0097306], response to farnesol [GO:0097307], response to perphenazine [GO:0097334], response to tetracycline [GO:1901326], response to rapamycin [GO:1901355], GO:1901422, response to propan-1-ol [GO:1901427], response to camptothecin [GO:1901563], response to docetaxel trihydrate [GO:1902519], response to doxorubicin [GO:1902520], GO:1902522, response to isobutanol [GO:1902665], response to dehydroepiandrosterone [GO:1903494], response to 11-deoxycorticosterone [GO:1903496], response to aldosterone [GO:1904044], response to forskolin [GO:1904321], response to diphenidol [GO:1904560], response to phorbol 13-acetate 12-myristate [GO:1904627], GO:1905092, response to haloperidol [GO:1905119] Relationships: is a type of response to oxygen-containing compound [GO:1901700] Also known as: process resulting in tolerance to alcohol Regulation: regulated by regulation of response to alcohol [GO:1901419]; negatively regulated by GO:1901420; positively regulated by positive regulation of response to alcohol [GO:1901421] Definition: Any process that results in a change in state or activity of a cell or an organism (in terms of movement, secretion, enzyme production, gene expression, etc.) as a result of an alcohol stimulus.